{
  "gene_name": "Regulator of G-protein signaling 14",
  "term_id": "GO:0051301",
  "gene_symbol": "RGS14",
  "gene": "UniProtKB:O43566",
  "term_label": "cell division"
}